{
  "gene_symbol": "PRORY",
  "term_label": "Unknown cellular component",
  "term_id": "UNKNOWN:0003",
  "gene_name": "Proline-rich protein, Y-linked",
  "gene": "UniProtKB:Q9H606"
}